{
  "gene": "UniProtKB:Q9NX47",
  "term_label": "ubiquitin protein ligase activity",
  "gene_symbol": "MARCHF5",
  "term_id": "GO:0061630",
  "gene_name": "E3 ubiquitin-protein ligase MARCHF5"
}